{
  "gene": "UniProtKB:Q9HD90",
  "term_id": "GO:0045944",
  "gene_name": "Neurogenic differentiation factor 4",
  "gene_symbol": "NEUROD4",
  "term_label": "positive regulation of transcription by RNA polymerase II"
}